{
  "term_label": "deadenylation-dependent decapping of nuclear-transcribed mRNA",
  "term_id": "GO:0000290",
  "gene_name": "m7GpppN-mRNA hydrolase",
  "gene_symbol": "DCP2",
  "gene": "UniProtKB:Q8IU60"
}